{
  "term_label": "apoptotic DNA fragmentation",
  "gene_name": "Nuclease EXOG, mitochondrial",
  "gene_symbol": "EXOG",
  "gene": "UniProtKB:Q9Y2C4",
  "term_id": "GO:0006309"
}